{
  "term_id": "GO:0009966",
  "gene_symbol": "KAZALD1",
  "gene": "UniProtKB:Q96I82",
  "gene_name": "Kazal-type serine protease inhibitor domain-containing protein 1",
  "term_label": "regulation of signal transduction"
}